{
  "term_id": "UNKNOWN:0003",
  "gene": "UniProtKB:P49441",
  "gene_symbol": "INPP1",
  "gene_name": "Inositol polyphosphate 1-phosphatase",
  "term_label": "Unknown cellular component"
}